{
  "term_id": "UNKNOWN:0003",
  "gene_symbol": "VHLL",
  "term_label": "Unknown cellular component",
  "gene_name": "von Hippel-Lindau-like protein",
  "gene": "UniProtKB:Q6RSH7"
}